{
  "gene_symbol": "FUNDC2",
  "term_id": "GO:0000422",
  "term_label": "autophagy of mitochondrion",
  "gene": "UniProtKB:Q9BWH2",
  "gene_name": "FUN14 domain-containing protein 2"
}